{
  "gene": "UniProtKB:Q8N122",
  "gene_name": "Regulatory-associated protein of mTOR",
  "term_id": "GO:0030307",
  "term_label": "positive regulation of cell growth",
  "gene_symbol": "RPTOR"
}